{
  "gene": "UniProtKB:Q9H061",
  "gene_name": "Transmembrane protein 126A",
  "gene_symbol": "TMEM126A",
  "term_id": "UNKNOWN:0001",
  "term_label": "Unknown molecular function"
}